negative regulation of response to formic acid [GO:1901461] (biological process) Also known as: down regulation of response to formic acid, down-regulation of response to formic acid, downregulation of response to formic acid, inhibition of response to formic acid Sources: GOC:TermGenie, GOC:mengo_curators Relationships: is a type of negative regulation of response to stimulus [GO:0048585]; is a type of regulation of response to formic acid [GO:1901460]; negatively regulates response to formic acid [GO:1901425] Definition: Any process that stops, prevents or reduces the frequency, rate or extent of response to formic acid.